{
  "term_id": "UNKNOWN:0003",
  "gene": "UniProtKB:Q8TBB5",
  "term_label": "Unknown cellular component",
  "gene_name": "Kelch domain-containing protein 4",
  "gene_symbol": "KLHDC4"
}